{
  "term_label": "neurogenesis",
  "term_id": "GO:0022008",
  "gene": "UniProtKB:Q9H4Q4",
  "gene_name": "PR domain zinc finger protein 12",
  "gene_symbol": "PRDM12"
}